penetration peg formation [GO:0075053] (biological process) References: PMID:26441323 Sources: GOC:pamgo_curators Also known as: initiation of symbiont penetration peg, symbiont penetration peg initiation, formation of symbiont penetration peg for entry into host, symbiont penetration peg formation for entry into host Definition: The assembly by the symbiont of a peg-like structure for the purpose of penetration into its host organism, which penetrates through the host cuticle and epidermal cell wall. The host is defined as the larger of the organisms involved in a symbiotic interaction. Regulation: regulated by modulation of penetration peg formation [GO:0075054]; positively regulated by positive regulation of penetration peg formation [GO:0075055] Note: Note that this term should not be used to annotate gene products of the host. It should only be used to annotate those gene products from the symbiont involved in this process. Relationships: is a type of formation of infection structure [GO:0075015]